{
  "gene_symbol": "CDH1",
  "term_label": "cell-cell junction assembly",
  "gene_name": "Cadherin-1",
  "term_id": "GO:0007043",
  "gene": "UniProtKB:P12830"
}